{
  "term_label": "positive regulation of coagulation",
  "gene_name": "Alpha-2-antiplasmin",
  "term_id": "GO:0050820",
  "gene_symbol": "SERPINF2",
  "gene": "UniProtKB:P08697"
}